regulation of immune complex clearance by monocytes and macrophages [GO:0090264] (BP) Sources: GOC:tb Relationships: is a type of regulation of immune effector process [GO:0002697]; regulates GO:0002436 Definition: Any process that modulates the rate, frequency, or extent of the process of immune complex clearance by monocytes or macrophages. Subtypes: positive regulation of immune complex clearance by monocytes and macrophages [GO:0090265]